{
  "term_label": "visual perception",
  "gene_name": "Cone cGMP-specific 3',5'-cyclic phosphodiesterase subunit alpha'",
  "term_id": "GO:0007601",
  "gene_symbol": "PDE6C",
  "gene": "UniProtKB:P51160"
}